{
  "gene": "UniProtKB:Q8N9Q2",
  "term_id": "UNKNOWN:0002",
  "term_label": "Unknown biological process",
  "gene_symbol": "SREK1IP1",
  "gene_name": "Protein SREK1IP1"
}